{
  "term_id": "GO:0005886",
  "gene": "UniProtKB:P29323",
  "term_label": "plasma membrane",
  "gene_name": "Ephrin type-B receptor 2",
  "gene_symbol": "EPHB2"
}